response to ecdysone [GO:0035075] (BP) Sources: GOC:bf Relationships: is a type of response to sterol [GO:0036314]; is a type of response to alcohol [GO:0097305]; is a type of response to ketone [GO:1901654] Subtypes: cellular response to ecdysone [GO:0071390] Definition: Any process that results in a change in state or activity of a cell or an organism (in terms of movement, secretion, enzyme production, gene expression, etc.) as a result of a ecdysone stimulus.